{
  "gene_name": "Sodium- and chloride-dependent GABA transporter 1",
  "gene_symbol": "SLC6A1",
  "gene": "UniProtKB:P30531",
  "term_label": "amino acid transport",
  "term_id": "GO:0006865"
}